{
  "term_label": "DNA-binding transcription factor activity, RNA polymerase II-specific",
  "term_id": "GO:0000981",
  "gene": "UniProtKB:P49335",
  "gene_name": "POU domain, class 3, transcription factor 4",
  "gene_symbol": "POU3F4"
}